{
  "term_id": "GO:0050000",
  "gene_symbol": "NDE1",
  "gene": "UniProtKB:Q9NXR1",
  "gene_name": "Nuclear distribution protein nudE homolog 1",
  "term_label": "chromosome localization"
}